{
  "gene_name": "DDB1- and CUL4-associated factor 12-like protein 2",
  "term_id": "UNKNOWN:0001",
  "gene_symbol": "DCAF12L2",
  "gene": "UniProtKB:Q5VW00",
  "term_label": "Unknown molecular function"
}